intermediate mesoderm development [GO:0048389] (biological process) Relationships: is a type of GO:0007498 Definition: The process whose specific outcome is the progression of the intermediate mesoderm over time, from its formation to the mature structure. The intermediate mesoderm is located between the lateral mesoderm and the paraxial mesoderm. It develops into the kidney and gonads. Sources: GOC:dgh